{
  "gene": "UniProtKB:O15514",
  "term_id": "GO:0006367",
  "gene_symbol": "POLR2D",
  "term_label": "transcription initiation at RNA polymerase II promoter",
  "gene_name": "DNA-directed RNA polymerase II subunit RPB4"
}